{
  "gene_symbol": "TRAV38-1",
  "term_label": "immune response",
  "gene_name": "T cell receptor alpha variable 38-1",
  "gene": "UniProtKB:A0A0B4J264",
  "term_id": "GO:0006955"
}